inferior raphe nucleus development [GO:0021724] (biological process) References: PMID:19003874 Sources: GOC:cjm, GOC:cls, GOC:curators, GOC:cvs, GOC:dgh Relationships: is a type of neural nucleus development [GO:0048857]; is part of GO:0021723 Also known as: inferior central nucleus development, posterior raphe nucleus development Definition: The process whose specific outcome is the progression of the inferior raphe nucleus over time, from its formation to the mature structure.